{
  "gene_symbol": "POPDC3",
  "gene": "UniProtKB:Q9HBV1",
  "gene_name": "Popeye domain-containing protein 3",
  "term_id": "GO:0042383",
  "term_label": "sarcolemma"
}